{
  "term_label": "cytoskeleton",
  "gene": "UniProtKB:P18206",
  "term_id": "GO:0005856",
  "gene_symbol": "VCL",
  "gene_name": "Vinculin"
}